{
  "gene_name": "Lysosomal thioesterase PPT2",
  "term_id": "UNKNOWN:0002",
  "gene": "UniProtKB:Q9UMR5",
  "gene_symbol": "PPT2",
  "term_label": "Unknown biological process"
}